{
  "gene_symbol": "SCYGR2",
  "gene_name": "Small cysteine and glycine repeat-containing protein 2",
  "term_label": "Unknown cellular component",
  "term_id": "UNKNOWN:0003",
  "gene": "UniProtKB:A0A286YFB4"
}